{
  "term_label": "membrane",
  "gene": "UniProtKB:Q13530",
  "gene_name": "Serine incorporator 3",
  "term_id": "GO:0016020",
  "gene_symbol": "SERINC3"
}